{
  "term_label": "mitochondrial respiratory chain complex I assembly",
  "term_id": "GO:0032981",
  "gene_symbol": "NDUFS5",
  "gene_name": "NADH dehydrogenase [ubiquinone] iron-sulfur protein 5",
  "gene": "UniProtKB:O43920"
}